positive regulation of phosphatidic acid biosynthetic process [GO:1905695] (biological process) Relationships: is a type of positive regulation of phospholipid biosynthetic process [GO:0071073]; is a type of GO:1905693; RO_0002213 phosphatidic acid biosynthetic process [GO:0006654] References: PMID:23767959 Sources: GOC:PARL, GOC:TermGenie, GOC:bc, GO_REF:0000058 Also known as: positive regulation of phosphatidic acid anabolism, positive regulation of phosphatidic acid biosynthesis, positive regulation of phosphatidic acid formation, positive regulation of phosphatidic acid synthesis, up regulation of phosphatidic acid anabolism, up regulation of phosphatidic acid biosynthesis, up regulation of phosphatidic acid biosynthetic process, up regulation of phosphatidic acid formation, up regulation of phosphatidic acid synthesis, up-regulation of phosphatidic acid anabolism, up-regulation of phosphatidic acid biosynthesis, up-regulation of phosphatidic acid biosynthetic process, up-regulation of phosphatidic acid formation, up-regulation of phosphatidic acid synthesis, upregulation of phosphatidic acid anabolism, upregulation of phosphatidic acid biosynthesis, upregulation of phosphatidic acid biosynthetic process, upregulation of phosphatidic acid formation, upregulation of phosphatidic acid synthesis, activation of phosphatidic acid anabolism, activation of phosphatidic acid biosynthesis, activation of phosphatidic acid biosynthetic process, activation of phosphatidic acid formation, activation of phosphatidic acid synthesis Definition: Any process that activates or increases the frequency, rate or extent of phosphatidic acid biosynthetic process.